{
  "gene_symbol": "MRPL2",
  "term_label": "RNA binding",
  "gene": "UniProtKB:Q5T653",
  "term_id": "GO:0003723",
  "gene_name": "Large ribosomal subunit protein uL2m"
}